{
  "term_id": "GO:0009966",
  "gene_symbol": "NCLN",
  "term_label": "regulation of signal transduction",
  "gene": "UniProtKB:Q969V3",
  "gene_name": "BOS complex subunit NCLN"
}